{
  "gene_symbol": "PRPF38B",
  "term_id": "UNKNOWN:0001",
  "gene": "UniProtKB:Q5VTL8",
  "gene_name": "Pre-mRNA-splicing factor 38B",
  "term_label": "Unknown molecular function"
}